{
  "gene_symbol": "PAK5",
  "term_label": "cytoplasm",
  "gene_name": "Serine_threonine-protein kinase PAK 5",
  "term_id": "GO:0005737",
  "gene": "UniProtKB:Q9P286"
}